regulation of skeletal muscle fiber development [GO:0048742] (biological process) Subtypes: positive regulation of skeletal muscle fiber development [GO:0048743], GO:0048744 Relationships: is_a regulation of myotube differentiation [GO:0010830]; is_a regulation of cell development [GO:0060284]; regulates skeletal muscle fiber development [GO:0048741] Sources: GOC:dph, GOC:jid, GOC:mtg_muscle, GOC:sm Definition: Any process that modulates the frequency, rate or extent of skeletal muscle fiber development. Muscle fibers are formed by the maturation of myotubes. They can be classed as slow, intermediate/fast or fast. Also known as: regulation of skeletal muscle fibre development, regulation of skeletal myofiber development, regulation of skeletal myofibre development